{
  "term_label": "Unknown molecular function",
  "gene": "UniProtKB:Q9Y462",
  "gene_symbol": "ZNF711",
  "gene_name": "Zinc finger protein 711",
  "term_id": "UNKNOWN:0001"
}